positive regulation of dendritic cell apoptotic process [GO:2000670] (biological process) Definition: Any process that activates or increases the frequency, rate or extent of dendritic cell apoptotic process. Sources: GOC:mtg_apoptosis, GOC:obol Also known as: positive regulation of dendritic cell apoptosis Relationships: is a type of positive regulation of leukocyte apoptotic process [GO:2000108]; is a type of regulation of dendritic cell apoptotic process [GO:2000668]; positively regulates GO:0097048